{
  "term_id": "GO:0030036",
  "gene_name": "Angiomotin",
  "term_label": "actin cytoskeleton organization",
  "gene": "UniProtKB:Q4VCS5",
  "gene_symbol": "AMOT"
}